{
  "term_label": "phosphatidylinositol phosphate binding",
  "term_id": "GO:1901981",
  "gene_symbol": "WASHC2C",
  "gene_name": "WASH complex subunit 2C",
  "gene": "UniProtKB:Q9Y4E1"
}